{
  "gene_name": "Protein SPT2 homolog",
  "term_label": "transcription by RNA polymerase I",
  "gene_symbol": "SPTY2D1",
  "gene": "UniProtKB:Q68D10",
  "term_id": "GO:0006360"
}